{
  "term_label": "cytosolic small ribosomal subunit",
  "gene_name": "Small ribosomal subunit protein uS15",
  "term_id": "GO:0022627",
  "gene_symbol": "RPS13",
  "gene": "UniProtKB:P62277"
}